{
  "term_label": "Unknown molecular function",
  "gene": "UniProtKB:Q0VAF6",
  "term_id": "UNKNOWN:0001",
  "gene_symbol": "SYCN",
  "gene_name": "Syncollin"
}